{
  "gene_symbol": "ZNF815P",
  "term_label": "Unknown molecular function",
  "term_id": "UNKNOWN:0001",
  "gene": "UniProtKB:A8K554",
  "gene_name": "Putative protein ZNF815"
}